{
  "gene_symbol": "PHTF1",
  "term_label": "Unknown molecular function",
  "gene_name": "Protein PHTF1",
  "gene": "UniProtKB:Q9UMS5",
  "term_id": "UNKNOWN:0001"
}